{
  "gene_name": "SLIT-ROBO Rho GTPase-activating protein 2C",
  "term_label": "negative regulation of cell migration",
  "gene": "UniProtKB:P0DJJ0",
  "term_id": "GO:0030336",
  "gene_symbol": "SRGAP2C"
}